{
  "gene_name": "Reticulon-1",
  "term_label": "brain development",
  "term_id": "GO:0007420",
  "gene": "UniProtKB:Q16799",
  "gene_symbol": "RTN1"
}